positive regulation of integrin activation [GO:0033625] (biological process) Sources: GOC:add Relationships: is a type of positive regulation of protein-containing complex assembly [GO:0031334]; is a type of regulation of integrin activation [GO:0033623]; RO_0002213 integrin activation [GO:0033622] Definition: Any process that activates or increases the frequency, rate, or extent of integrin activation. Also known as: positive regulation of integrin complex activation Subtypes: positive regulation of integrin activation by cell surface receptor linked signal transduction [GO:0033626]